negative regulation of cardiac chamber morphogenesis [GO:1901220] (biological process) Also known as: down regulation of cardiac chamber morphogenesis, down regulation of heart chamber morphogenesis, down-regulation of cardiac chamber morphogenesis, down-regulation of heart chamber morphogenesis, downregulation of cardiac chamber morphogenesis, downregulation of heart chamber morphogenesis, negative regulation of heart chamber morphogenesis, inhibition of cardiac chamber morphogenesis, inhibition of heart chamber morphogenesis Sources: GOC:BHF, GOC:TermGenie Relationships: is a type of negative regulation of developmental process [GO:0051093]; is a type of GO:1901219; negatively regulates cardiac chamber morphogenesis [GO:0003206] Definition: Any process that stops, prevents or reduces the frequency, rate or extent of cardiac chamber morphogenesis.